{
  "term_label": "forebrain development",
  "term_id": "GO:0030900",
  "gene": "UniProtKB:Q8NBI3",
  "gene_name": "Draxin",
  "gene_symbol": "DRAXIN"
}